cell-cell adhesion [GO:0098609] (biological process) Subtypes: endocardial cushion fusion [GO:0003274], cell-cell adhesion involved in ameboidal cell migration [GO:0003367], homophilic cell-cell adhesion [GO:0007156], heterophilic cell-cell adhesion [GO:0007157], GO:0007158, leukocyte cell-cell adhesion [GO:0007159], pollen tube adhesion [GO:0009865], pollen adhesion [GO:0009876], calcium-independent cell-cell adhesion [GO:0016338], calcium-dependent cell-cell adhesion [GO:0016339], neuronal-glial interaction involved in cerebral cortex radial glia guided migration [GO:0021812], cell-cell adhesion involved in neuronal-glial interactions involved in cerebral cortex radial glia guided migration [GO:0021813], cell-cell adhesion involved in cerebral cortex tangential migration using cell-cell interactions [GO:0021832], neuronal-glial interaction involved in hindbrain glial-mediated radial cell migration [GO:0021944], cell-cell adhesion mediated by integrin [GO:0033631], homotypic cell-cell adhesion [GO:0034109], heterotypic cell-cell adhesion [GO:0034113], GO:0044331, cell-cell adhesion involved in sealing an epithelial fold [GO:0060607], mesenchymal cell condensation involved in mammary fat development [GO:0060647], chorio-allantoic fusion [GO:0060710], GO:0070586, pre-tubular aggregate formation [GO:0072035], cell-cell adhesion involved in synapse maturation [GO:0090125], epithelial cell-cell adhesion [GO:0090136], regulation of actin cytoskeleton organization by cell-cell adhesion [GO:0090138], cell-cell adhesion involved in establishment of planar polarity [GO:0090250], adhesion between unicellular organisms [GO:0098610], synaptic membrane adhesion [GO:0099560], cell-cell adhesion in response to extracellular stimulus [GO:0140039] Regulation: regulated by regulation of cell-cell adhesion [GO:0022407]; negatively regulated by negative regulation of cell-cell adhesion [GO:0022408]; positively regulated by GO:0022409 Also known as: single organismal cell-cell adhesion Definition: The attachment of one cell to another cell via adhesion molecules. Relationships: is a type of cell adhesion [GO:0007155] Sources: GOC:dos